{
  "gene_name": "Complement C5",
  "gene": "UniProtKB:P01031",
  "gene_symbol": "C5",
  "term_label": "Unknown cellular component",
  "term_id": "UNKNOWN:0003"
}